{
  "term_id": "GO:0008540",
  "gene_symbol": "PSMD4",
  "gene": "UniProtKB:P55036",
  "gene_name": "26S proteasome non-ATPase regulatory subunit 4",
  "term_label": "proteasome regulatory particle, base subcomplex"
}